{
  "gene_symbol": "CT47A12",
  "gene_name": "Cancer_testis antigen 47A",
  "term_id": "UNKNOWN:0002",
  "gene": "UniProtKB:Q5JQC4",
  "term_label": "Unknown biological process"
}